right ventricular compact myocardium morphogenesis [GO:0003226] (biological process) Definition: The process in which the anatomical structures of the right ventricular compact myocardium are generated and organized. Relationships: is a type of right ventricular cardiac muscle tissue morphogenesis [GO:0003221]; is a type of ventricular compact myocardium morphogenesis [GO:0003223] Sources: GOC:mtg_heart